{
  "term_id": "UNKNOWN:0001",
  "gene_name": "Multiple epidermal growth factor-like domains protein 9",
  "term_label": "Unknown molecular function",
  "gene_symbol": "MEGF9",
  "gene": "UniProtKB:Q9H1U4"
}